{
  "gene_symbol": "CLN6",
  "gene": "UniProtKB:Q9NWW5",
  "term_label": "membrane",
  "gene_name": "Ceroid-lipofuscinosis neuronal protein 6",
  "term_id": "GO:0016020"
}